{
  "gene": "UniProtKB:Q15788",
  "term_label": "cellular response to hormone stimulus",
  "gene_name": "Nuclear receptor coactivator 1",
  "term_id": "GO:0032870",
  "gene_symbol": "NCOA1"
}